{
  "term_label": "cell-cell adhesion",
  "term_id": "GO:0098609",
  "gene_name": "Immunoglobulin superfamily member 5",
  "gene": "UniProtKB:Q9NSI5",
  "gene_symbol": "IGSF5"
}